ATP binding [GO:0005524] (molecular function) Sources: ISBN:0198506732 Definition: Binding to ATP, adenosine 5'-triphosphate, a universally important coenzyme and enzyme regulator. Regulation: positively regulated by adenyl-nucleotide exchange factor activity [GO:0000774] Relationships: is a type of GO:0032559; is a type of purine ribonucleoside triphosphate binding [GO:0035639] Also known as: Mg-ATP binding, MgATP binding